regulation of neutrophil mediated killing of gram-negative bacterium [GO:0070951] (biological process) Definition: Any process that modulates the rate, frequency or extent of neutrophil mediated killing of a gram-negative bacterium, the directed killing of a gram-negative bacterium by a neutrophil. Sources: GOC:add, GOC:mah Relationships: is a type of regulation of neutrophil mediated killing of bacterium [GO:0070950]; regulates neutrophil-mediated killing of gram-negative bacterium [GO:0070945] Subtypes: negative regulation of neutrophil mediated killing of gram-negative bacterium [GO:0070957], positive regulation of neutrophil mediated killing of gram-negative bacterium [GO:0070963]